{
  "gene_symbol": "PRELID2",
  "term_label": "phospholipid transport",
  "gene": "UniProtKB:Q8N945",
  "term_id": "GO:0015914",
  "gene_name": "PRELI domain-containing protein 2"
}